regulation of spindle attachment to meiosis I kinetochore [GO:1904967] (biological process) Definition: Any process that modulates the frequency, rate or extent of attachment of spindle microtubules to kinetochore involved in homologous chromosome segregation. Subtypes: positive regulation of spindle attachment to meiosis I kinetochore [GO:1904968] Relationships: is a type of GO:0051988; is a type of repair of kinetochore microtubule attachment defect [GO:0140274]; is a type of meiotic cell cycle process [GO:1903046]; is a type of regulation of reproductive process [GO:2000241]; is part of meiotic metaphase I homologous chromosome alignment [GO:0043060]; regulates spindle attachment to meiosis I kinetochore [GO:0051455] Also known as: regulation of attachment of spindle microtubules to kinetochore involved in homologous chromosome segregation, regulation of attachment of spindle microtubules to kinetochore involved in meiosis I, regulation of monopolar attachment, regulation of sister kinetochore mono-orientation, correction of merotelic kinetochore attachment, meiosis I, regulation of attachment of spindle microtubules to kinetochore during meiosis I, repair of merotelic kinetochore attachment defect, meiosis I References: PMID:21920317, PMID:23770679 Sources: GOC:TermGenie, GOC:vw, GO_REF:0000058